{
  "gene_name": "Olfactory receptor 4F3_4F16_4F29",
  "gene": "UniProtKB:Q6IEY1",
  "term_id": "UNKNOWN:0003",
  "term_label": "Unknown cellular component",
  "gene_symbol": "OR4F16"
}